protein kinase inhibitor activity [GO:0004860] (molecular function) Subtypes: protein serine/threonine kinase inhibitor activity [GO:0030291], protein tyrosine kinase inhibitor activity [GO:0030292] Definition: Binds to and stops, prevents or reduces the activity of a protein kinase. Sources: GOC:ai Relationships: is a type of kinase inhibitor activity [GO:0019210]; is_a protein kinase regulator activity [GO:0019887]; negatively regulates protein kinase activity [GO:0004672]